{
  "gene_name": "Follicle-stimulating hormone receptor",
  "term_label": "follicle-stimulating hormone signaling pathway",
  "gene": "UniProtKB:P23945",
  "term_id": "GO:0042699",
  "gene_symbol": "FSHR"
}